muconolactone delta-isomerase activity [GO:0016159] (molecular function) Relationships: is a type of GO:0016863 Sources: RHEA:12348 Also known as: muconolactone D-isomerase activity, 5-oxo-4,5-dihydrofuran-2-acetate delta3-delta2-isomerase activity, muconolactone isomerase activity Definition: Catalysis of the reaction: (S)-muconolactone = (4,5-dihydro-5-oxofuran-2-yl)-acetate.